{
  "term_id": "GO:0090110",
  "term_label": "COPII-coated vesicle cargo loading",
  "gene_name": "Protein transport protein Sec31A",
  "gene": "UniProtKB:O94979",
  "gene_symbol": "SEC31A"
}